{
  "gene_name": "52 kDa repressor of the inhibitor of the protein kinase",
  "gene": "UniProtKB:O43422",
  "term_label": "Unknown biological process",
  "gene_symbol": "THAP12",
  "term_id": "UNKNOWN:0002"
}